{
  "term_id": "GO:0005681",
  "gene": "UniProtKB:Q9NVM6",
  "term_label": "spliceosomal complex",
  "gene_name": "DnaJ homolog subfamily C member 17",
  "gene_symbol": "DNAJC17"
}